myoblast fate specification involved in skeletal muscle regeneration [GO:0014838] (BP) References: PMID:16607119 Sources: CL:0000056, GOC:ef, GOC:mtg_muscle Definition: The process in which a satellite cell becomes capable of differentiating autonomously into a myoblast in an environment that is neutral with respect to the developmental pathway. Upon specification, the cell fate can be reversed. This occurs as part of skeletal muscle regeneration. A myoblast is a mononucleate cell type that, by fusion with other myoblasts, gives rise to the myotubes that eventually develop into skeletal muscle fibers. Relationships: is a type of myoblast fate specification [GO:0048626]; BFO_0000050 myoblast fate commitment involved in skeletal muscle regeneration [GO:0014836]